{
  "gene_symbol": "PGLYRP1",
  "gene_name": "Peptidoglycan recognition protein 1",
  "gene": "UniProtKB:O75594",
  "term_label": "defense response to Gram-positive bacterium",
  "term_id": "GO:0050830"
}